{
  "gene": "UniProtKB:P0C7V9",
  "term_label": "rRNA (cytosine-N4-)-methyltransferase activity",
  "gene_symbol": "METTL15P1",
  "gene_name": "Putative methyltransferase-like protein 15P1",
  "term_id": "GO:0071424"
}